{
  "term_id": "GO:0043130",
  "term_label": "ubiquitin binding",
  "gene_name": "UBX domain-containing protein 2B",
  "gene": "UniProtKB:Q14CS0",
  "gene_symbol": "UBXN2B"
}